{
  "gene_name": "Protocadherin gamma-B3",
  "gene_symbol": "PCDHGB3",
  "term_id": "GO:0007155",
  "term_label": "cell adhesion",
  "gene": "UniProtKB:Q9Y5G1"
}